positive regulation of cell fate specification [GO:0042660] (biological process) Relationships: is a type of positive regulation of cell fate commitment [GO:0010455]; is a type of regulation of cell fate specification [GO:0042659]; positively regulates GO:0001708 Also known as: up regulation of cell fate specification, up-regulation of cell fate specification, upregulation of cell fate specification, activation of cell fate specification, stimulation of cell fate specification Sources: GOC:go_curators Definition: Any process that activates or enables a cell to adopt a specific fate. Subtypes: positive regulation of atrichoblast fate specification [GO:0010059], positive regulation of trichoblast fate specification [GO:0010063], positive regulation of mesodermal cell fate specification [GO:0048337], positive regulation of neural crest cell fate specification [GO:1905297]